{
  "gene_name": "Muscarinic acetylcholine receptor M3",
  "term_label": "G protein-coupled receptor signaling pathway, coupled to cyclic nucleotide second messenger",
  "term_id": "GO:0007187",
  "gene": "UniProtKB:P20309",
  "gene_symbol": "CHRM3"
}